{
  "term_label": "cytoplasm",
  "gene_name": "Serine_threonine-protein phosphatase 4 regulatory subunit 1",
  "term_id": "GO:0005737",
  "gene_symbol": "PPP4R1",
  "gene": "UniProtKB:Q8TF05"
}